protein acetylation [GO:0006473] (biological process) Regulation: regulated by regulation of protein acetylation [GO:1901983]; negatively regulated by GO:1901984; positively regulated by positive regulation of protein acetylation [GO:1901985] Definition: The addition of an acetyl group to a protein amino acid. An acetyl group is CH3CO-, derived from acetic [ethanoic] acid. Also known as: protein amino acid acetylation Relationships: is a type of protein acylation [GO:0043543] Sources: GOC:ai Subtypes: GO:0006474, internal protein amino acid acetylation [GO:0006475], peptidyl-lysine acetylation [GO:0018394], peptidyl-cysteine acetylation [GO:0018533], peptidyl-serine acetylation [GO:0030920], post-translational protein acetylation [GO:0034421], peptidyl-threonine acetylation [GO:0120257]